cell-substrate junction [GO:0030055] (cellular component) Relationships: is a type of anchoring junction [GO:0070161] References: PMID:10419689, PMID:1643657, PMID:16805308, PMID:26923917, PMID:8314002 Sources: GOC:aruk, GOC:bc, GOC:hb, GOC:mah Definition: A cell junction that forms a connection between a cell and the extracellular matrix. Also known as: cell-matrix junction Subtypes: GO:0005925, GO:0005927, hemidesmosome [GO:0030056]